exogenous antibiotic catabolic process [GO:0042740] (BP) Definition: The chemical reactions and pathways resulting in the breakdown of an antibiotic that has originated externally to the cell or organism. Relationships: is a type of antibiotic catabolic process [GO:0017001]; is a type of xenobiotic catabolic process [GO:0042178]; BFO_0000050 response to antibiotic [GO:0046677] Also known as: exogenous antibiotic breakdown, exogenous antibiotic catabolism, exogenous antibiotic degradation Sources: GOC:jl